citrate (pro-3S)-lyase activity [GO:0008815] (molecular function) Sources: RHEA:10760 Also known as: citrate lyase activity, citrate lyase, citrase activity, citratase activity, citrate aldolase activity, citrate oxaloacetate-lyase [(pro-3S)-CH2COO-->acetate], citrate oxaloacetate-lyase activity, citric aldolase activity, citridesmolase activity, citritase activity Definition: Catalysis of the reaction: citrate = acetate + oxaloacetate. Relationships: is_a oxo-acid-lyase activity [GO:0016833]